{
  "gene_symbol": "ZNF33B",
  "gene": "UniProtKB:Q06732",
  "term_id": "GO:0005634",
  "gene_name": "Zinc finger protein 33B",
  "term_label": "nucleus"
}